E.F.G complex [GO:0034692] (cellular component) References: PMID:8641291 Definition: A protein complex that comprises three core spliceosomal proteins, designated E, F, and G. Formation of the E.F.G complex is essential but not sufficient for the formation of a stable U1 snRNP complex. Relationships: is a type of nuclear protein-containing complex [GO:0140513]